{
  "term_id": "GO:0005634",
  "term_label": "nucleus",
  "gene_symbol": "METTL18",
  "gene": "UniProtKB:O95568",
  "gene_name": "Histidine protein methyltransferase 1 homolog"
}